{
  "gene_symbol": "AGFG1",
  "term_label": "cytoplasmic vesicle",
  "term_id": "GO:0031410",
  "gene": "UniProtKB:P52594",
  "gene_name": "Arf-GAP domain and FG repeat-containing protein 1"
}